phytosteroid catabolic process [GO:0016130] (biological process) Relationships: is a type of steroid catabolic process [GO:0006706] Subtypes: GO:0016133 Definition: The chemical reactions and pathways resulting in the breakdown of phytosteroids, steroids that differ from animal steroids in having substitutions at C24 and/or a double bond at C22. Phytosteroids are so named because they occur in higher plants; some, notably ergosterol, are also found in fungi. Also known as: phytosteroid breakdown, phytosteroid catabolism, phytosteroid degradation Sources: GOC:go_curators, GOC:mah